{
  "gene_symbol": "DHX32",
  "term_label": "helicase activity",
  "gene": "UniProtKB:Q7L7V1",
  "gene_name": "Putative pre-mRNA-splicing factor ATP-dependent RNA helicase DHX32",
  "term_id": "GO:0004386"
}